CD4-positive, alpha-beta T cell proliferation [GO:0035739] (biological process) Relationships: is_a CD4-positive, alpha-beta T cell activation [GO:0035710]; is a type of alpha-beta T cell proliferation [GO:0046633] Definition: The expansion of a CD4-positive, alpha-beta T cell population by cell division. Regulation: regulated by regulation of CD4-positive, alpha-beta T cell proliferation [GO:2000561]; negatively regulated by GO:2000562; positively regulated by positive regulation of CD4-positive, alpha-beta T cell proliferation [GO:2000563] Subtypes: activated CD4-positive, alpha-beta T cell proliferation [GO:0035741] Sources: CL:0000624, GOC:BHF